naphthalenesulfonate metabolic process [GO:0018984] (biological process) Also known as: naphthalenesulfonate metabolism, naphthalenesulphonate metabolic process, naphthalenesulphonate metabolism Definition: The chemical reactions and pathways involving naphthalenesulfonate, sulfonated derivatives of naphthalene. Relationships: is a type of organic acid metabolic process [GO:0006082]; is a type of sulfur compound metabolic process [GO:0006790] Sources: GOC:ai